thiamine pyridinylase activity [GO:0050332] (MF) Sources: EC:2.5.1.2, RHEA:17697 Relationships: is a type of transferase activity, transferring alkyl or aryl (other than methyl) groups [GO:0016765] Also known as: thiamin pyridinylase activity, thiaminase I activity, pyrimidine transferase activity, thiamin hydrolase activity, thiamin pyridinolase activity, thiamin:base 2-methyl-4-aminopyrimidine-5-methenyltransferase activity, thiamine hydrolase activity, thiamine pyridinolase activity, thiamine:base 2-methyl-4-aminopyrimidine-5-methenyltransferase activity Definition: Catalysis of the reaction: pyridine + thiamine = 5-(2-hydroxyethyl)-4-methylthiazole + heteropyrithiamine.